{
  "gene_name": "Interferon-induced transmembrane protein 10",
  "gene": "UniProtKB:A6NMD0",
  "term_id": "UNKNOWN:0001",
  "term_label": "Unknown molecular function",
  "gene_symbol": "IFITM10"
}